{
  "term_id": "GO:0000049",
  "gene_symbol": "SARS1",
  "gene": "UniProtKB:P49591",
  "term_label": "tRNA binding",
  "gene_name": "Serine--tRNA ligase, cytoplasmic"
}